regulation of cytotoxic T cell degranulation [GO:0043317] (biological process) Definition: Any process that modulates the frequency, rate, or extent of cytotoxic T cell degranulation. Sources: ISBN:0781735149 Also known as: regulation of cytotoxic T cell granule exocytosis, regulation of cytotoxic T lymphocyte degranulation, regulation of cytotoxic T lymphocyte granule exocytosis, regulation of cytotoxic T-cell degranulation, regulation of cytotoxic T-cell granule exocytosis, regulation of cytotoxic T-lymphocyte degranulation, regulation of cytotoxic T-lymphocyte granule exocytosis Relationships: is a type of regulation of T cell mediated cytotoxicity [GO:0001914]; is a type of regulation of leukocyte degranulation [GO:0043300]; regulates cytotoxic T cell degranulation [GO:0043316] Subtypes: negative regulation of cytotoxic T cell degranulation [GO:0043318], positive regulation of cytotoxic T cell degranulation [GO:0043319]